{
  "gene": "UniProtKB:Q15620",
  "gene_name": "Olfactory receptor 8B8",
  "term_label": "olfactory receptor activity",
  "term_id": "GO:0004984",
  "gene_symbol": "OR8B8"
}